{
  "gene": "UniProtKB:Q6P9F7",
  "term_label": "aspartate transmembrane transport",
  "gene_name": "Volume-regulated anion channel subunit LRRC8B",
  "gene_symbol": "LRRC8B",
  "term_id": "GO:0015810"
}